{
  "term_label": "signal transduction",
  "term_id": "GO:0007165",
  "gene_symbol": "OLFM2",
  "gene_name": "Noelin-2",
  "gene": "UniProtKB:O95897"
}